{
  "term_label": "Unknown molecular function",
  "term_id": "UNKNOWN:0001",
  "gene": "UniProtKB:Q9BXB1",
  "gene_name": "Leucine-rich repeat-containing G-protein coupled receptor 4",
  "gene_symbol": "LGR4"
}